{
  "term_label": "nucleus",
  "term_id": "GO:0005634",
  "gene_name": "Mitochondrial-derived peptide MOTS-c",
  "gene_symbol": "MT-RNR1",
  "gene": "UniProtKB:A0A0C5B5G6"
}